{
  "gene_symbol": "NEU2",
  "gene_name": "Sialidase-2",
  "term_id": "GO:0006689",
  "gene": "UniProtKB:Q9Y3R4",
  "term_label": "ganglioside catabolic process"
}